protein-N(PI)-phosphohistidine-beta-glucoside phosphotransferase system transporter activity [GO:0022882] (MF) Also known as: beta-glucoside PTS transporter activity Relationships: is a type of GO:0008982; is a type of beta-glucoside transmembrane transporter activity [GO:0015573] Sources: GOC:mtg_transport, ISBN:0815340729 Definition: Catalysis of the PEP-dependent, phosphoryl transfer-driven transport of substances across a membrane. The transport happens by catalysis of the reaction: protein N-phosphohistidine + beta-glucoside(out) = protein histidine + beta-glucoside phosphate(in). This differs from primary and secondary active transport in that the solute is modified during transport.